positive regulation of myotube cell migration [GO:0110124] (biological process) Relationships: is a type of positive regulation of cell migration [GO:0030335]; is a type of GO:0110123; positively regulates myotube cell migration [GO:0110122] Definition: Any process that activates, maintains or increases the frequency, rate or extent of myotube cell migration. References: PMID:29122742 Sources: GOC:ha